rRNA pseudouridylation guide activity [GO:0030559] (molecular function) Note: Note that this term describes the activity of a nucleic acid, usually RNA, gene product that interacts with other RNA molecules via base pairing; it should not be used to annotate proteins. Relationships: is a type of rRNA modification guide activity [GO:0030556]; is a type of RNA pseudouridylation guide activity [GO:0030558] References: PMID:12457565 Sources: GOC:mah Definition: Specifies the site of pseudouridylation in an rRNA molecule by base pairing with a short sequence around the target residue.